{
  "term_label": "G protein-coupled glutamate receptor signaling pathway",
  "term_id": "GO:0007216",
  "gene_name": "Metabotropic glutamate receptor 3",
  "gene": "UniProtKB:Q14832",
  "gene_symbol": "GRM3"
}